{
  "term_label": "Unknown biological process",
  "gene_name": "Large ribosomal subunit protein mL43",
  "gene": "UniProtKB:Q8N983",
  "gene_symbol": "MRPL43",
  "term_id": "UNKNOWN:0002"
}